{
  "gene": "UniProtKB:P21817",
  "term_id": "GO:0033017",
  "term_label": "sarcoplasmic reticulum membrane",
  "gene_symbol": "RYR1",
  "gene_name": "Ryanodine receptor 1"
}